{
  "term_label": "microtubule organizing center",
  "term_id": "GO:0005815",
  "gene_symbol": "DCDC2C",
  "gene": "UniProtKB:A8MYV0",
  "gene_name": "Doublecortin domain-containing protein 2C"
}